{
  "term_id": "UNKNOWN:0002",
  "term_label": "Unknown biological process",
  "gene_symbol": "FAM151A",
  "gene": "UniProtKB:Q8WW52",
  "gene_name": "Protein FAM151A"
}